{
  "term_id": "GO:0045088",
  "gene_symbol": "CD300A",
  "gene": "UniProtKB:Q9UGN4",
  "gene_name": "CMRF35-like molecule 8",
  "term_label": "regulation of innate immune response"
}